{
  "term_label": "plasma membrane",
  "gene": "UniProtKB:O75128",
  "term_id": "GO:0005886",
  "gene_name": "Protein cordon-bleu",
  "gene_symbol": "COBL"
}